negative regulation of intraciliary anterograde transport [GO:1905797] (biological process) Relationships: is a type of negative regulation of intracellular transport [GO:0032387]; is a type of regulation of intraciliary anterograde transport [GO:1905796]; negatively regulates intraciliary anterograde transport [GO:0035720] Definition: Any process that stops, prevents or reduces the frequency, rate or extent of intraciliary anterograde transport. Also known as: down regulation of intraciliary anterograde transport, down regulation of intraflagellar anterograde transport, down-regulation of intraciliary anterograde transport, down-regulation of intraflagellar anterograde transport, downregulation of intraciliary anterograde transport, downregulation of intraflagellar anterograde transport, negative regulation of intraflagellar anterograde transport, inhibition of intraciliary anterograde transport, inhibition of intraflagellar anterograde transport References: PMID:27930654 Sources: GOC:TermGenie, GO_REF:0000058